positive regulation of toll-like receptor 2 signaling pathway [GO:0034137] (biological process) Relationships: is a type of GO:0034135; is a type of GO:0062208; positively regulates GO:0034134 References: PMID:16551253, PMID:17328678 Sources: GOC:add Definition: Any process that activates or increases the frequency, rate, or extent of toll-like receptor 2 signaling pathway. Also known as: positive regulation of TLR2 signaling pathway, positive regulation of toll-like receptor 2 signalling pathway